{
  "gene": "UniProtKB:Q9GZQ6",
  "gene_name": "Neuropeptide FF receptor 1",
  "term_id": "GO:0032870",
  "gene_symbol": "NPFFR1",
  "term_label": "cellular response to hormone stimulus"
}